galactose catabolic process [GO:0019388] (biological process) Subtypes: galactose catabolic process via D-galactonate [GO:0033498], galactose catabolic process via UDP-galactose, Leloir pathway [GO:0033499], glycolytic process from galactose [GO:0061623], beta-D-galactofuranose catabolic process [GO:1901357] Also known as: galactose breakdown, galactose catabolism, galactose degradation Definition: The chemical reactions and pathways resulting in the breakdown of galactose, the aldohexose galacto-hexose. Relationships: is a type of galactose metabolic process [GO:0006012]; is a type of hexose catabolic process [GO:0019320] Sources: ISBN:0198506732